{
  "gene": "UniProtKB:Q8TDW0",
  "gene_name": "Volume-regulated anion channel subunit LRRC8C",
  "term_id": "GO:0005737",
  "gene_symbol": "LRRC8C",
  "term_label": "cytoplasm"
}